{
  "gene_name": "Cytosolic carboxypeptidase-like protein 5",
  "term_label": "tubulin binding",
  "gene": "UniProtKB:Q8NDL9",
  "term_id": "GO:0015631",
  "gene_symbol": "AGBL5"
}